{
  "term_label": "DNA-binding transcription repressor activity, RNA polymerase II-specific",
  "term_id": "GO:0001227",
  "gene_name": "Zinc finger and BTB domain-containing protein 32",
  "gene_symbol": "ZBTB32",
  "gene": "UniProtKB:Q9Y2Y4"
}